{
  "term_label": "mitochondrion",
  "gene_name": "Peroxiredoxin-5, mitochondrial",
  "gene_symbol": "PRDX5",
  "gene": "UniProtKB:P30044",
  "term_id": "GO:0005739"
}